{
  "gene": "UniProtKB:Q9Y235",
  "term_id": "GO:0005737",
  "gene_symbol": "APOBEC2",
  "gene_name": "C-U-editing enzyme APOBEC-2",
  "term_label": "cytoplasm"
}